{
  "gene_name": "Polycystin-1",
  "term_label": "calcium ion transport",
  "gene": "UniProtKB:P98161",
  "term_id": "GO:0006816",
  "gene_symbol": "PKD1"
}